{
  "gene_symbol": "RAB35",
  "term_id": "GO:0005886",
  "term_label": "plasma membrane",
  "gene_name": "Ras-related protein Rab-35",
  "gene": "UniProtKB:Q15286"
}